renal interstitial fibroblast development [GO:0072141] (biological process) Sources: GOC:mtg_kidney_jan10 Relationships: is a type of cell development [GO:0048468]; is part of kidney interstitial fibroblast differentiation [GO:0072071] Also known as: kidney interstitial cell development Definition: The process whose specific outcome is the progression of a renal interstitial fibroblast over time, from its formation to the mature structure. Subtypes: mesonephric interstitial fibroblast development [GO:0061267], metanephric interstitial fibroblast development [GO:0072259]